{
  "gene_name": "D-amino-acid oxidase",
  "gene_symbol": "DAO",
  "term_label": "peroxisomal matrix",
  "gene": "UniProtKB:P14920",
  "term_id": "GO:0005782"
}